{
  "term_label": "modulation of chemical synaptic transmission",
  "term_id": "GO:0050804",
  "gene_name": "Glutamate receptor ionotropic, kainate 1",
  "gene_symbol": "GRIK1",
  "gene": "UniProtKB:P39086"
}